vasodilation [GO:0042311] (BP) Sources: GOC:pr, ISBN:0192800981 Relationships: is a type of blood vessel diameter maintenance [GO:0097746] Subtypes: artery vasodilation involved in baroreceptor response to increased systemic arterial blood pressure [GO:0001984], norepinephrine-epinephrine-mediated vasodilation involved in regulation of systemic arterial blood pressure [GO:0002025], angiotensin-mediated vasodilation involved in regulation of systemic arterial blood pressure [GO:0002033], vasodilation involved in acute inflammatory response [GO:0002527], acetylcholine-mediated vasodilation involved in regulation of systemic arterial blood pressure [GO:0003069], epinephrine-mediated vasodilation [GO:0003121], norepinephrine-mediated vasodilation [GO:0003122] Also known as: positive regulation of blood vessel size, vasodilatation Definition: An increase in the internal diameter of blood vessels, especially arterioles or capillaries, due to relaxation of smooth muscle cells that line the vessels, and usually resulting in a decrease in blood pressure.